{
  "term_id": "GO:0007605",
  "term_label": "sensory perception of sound",
  "gene_symbol": "OTOS",
  "gene": "UniProtKB:Q8NHW6",
  "gene_name": "Otospiralin"
}